{
  "gene_name": "Solute carrier family 49 member 4",
  "gene": "UniProtKB:Q96SL1",
  "term_label": "Unknown molecular function",
  "term_id": "UNKNOWN:0001",
  "gene_symbol": "SLC49A4"
}